DNA polymerase III, clamp loader complex [GO:0043846] (cellular component) Definition: A heptamer that includes the tau and gamma products of the dnaX gene and the chi/psi subcomplex. Confers structural asymmetry that allows the polymerase to replicate both leading and lagging strands. References: PMID:12940977 Also known as: clamp loader complex, DNA polymerase III, DnaX complex, DNA polymerase III, DnaX subcomplex Relationships: is a type of nuclear protein-containing complex [GO:0140513]; is part of GO:0009360